{
  "term_id": "UNKNOWN:0002",
  "gene": "UniProtKB:Q5SRI9",
  "term_label": "Unknown biological process",
  "gene_name": "Glycoprotein endo-alpha-1,2-mannosidase",
  "gene_symbol": "MANEA"
}